{
  "term_label": "glycosylceramidase activity",
  "term_id": "GO:0017042",
  "gene_name": "Cytosolic beta-glucosidase",
  "gene_symbol": "GBA3",
  "gene": "UniProtKB:Q9H227"
}